{
  "term_id": "GO:0005739",
  "gene_symbol": "MT-CO3",
  "gene_name": "Cytochrome c oxidase subunit 3",
  "term_label": "mitochondrion",
  "gene": "UniProtKB:P00414"
}